{
  "gene": "UniProtKB:O75581",
  "gene_symbol": "LRP6",
  "gene_name": "Low-density lipoprotein receptor-related protein 6",
  "term_label": "Unknown molecular function",
  "term_id": "UNKNOWN:0001"
}